{
  "term_id": "GO:0005634",
  "gene_name": "Hepatocyte nuclear factor 1-alpha",
  "gene": "UniProtKB:P20823",
  "gene_symbol": "HNF1A",
  "term_label": "nucleus"
}